{
  "gene_name": "Coiled-coil domain-containing protein 38",
  "gene_symbol": "CCDC38",
  "term_label": "Unknown biological process",
  "gene": "UniProtKB:Q502W7",
  "term_id": "UNKNOWN:0002"
}